{
  "term_label": "negative regulation of DNA-templated transcription",
  "gene_name": "Brain acid soluble protein 1",
  "gene_symbol": "BASP1",
  "term_id": "GO:0045892",
  "gene": "UniProtKB:P80723"
}